{
  "gene_name": "Olfactory receptor 10J5",
  "gene_symbol": "OR10J5",
  "term_id": "GO:0004984",
  "gene": "UniProtKB:Q8NHC4",
  "term_label": "olfactory receptor activity"
}